{
  "gene_name": "cTAGE family member 2",
  "gene": "UniProtKB:Q96RT6",
  "term_label": "Unknown molecular function",
  "term_id": "UNKNOWN:0001",
  "gene_symbol": "CTAGE1"
}